{
  "term_id": "GO:0032956",
  "gene": "UniProtKB:Q17R89",
  "gene_name": "Rho GTPase-activating protein 44",
  "term_label": "regulation of actin cytoskeleton organization",
  "gene_symbol": "ARHGAP44"
}